{
  "term_label": "regulation of transcription by RNA polymerase II",
  "gene": "UniProtKB:Q13360",
  "gene_name": "Zinc finger protein 177",
  "gene_symbol": "ZNF177",
  "term_id": "GO:0006357"
}